{
  "term_id": "GO:0043005",
  "term_label": "neuron projection",
  "gene": "UniProtKB:Q70Z44",
  "gene_symbol": "HTR3D",
  "gene_name": "5-hydroxytryptamine receptor 3D"
}